{
  "term_label": "nucleus",
  "gene": "UniProtKB:P10243",
  "gene_name": "Myb-related protein A",
  "gene_symbol": "MYBL1",
  "term_id": "GO:0005634"
}